regulation of hypoxia-inducible factor-1alpha signaling pathway [GO:1902071] (biological process) Definition: Any process that modulates the frequency, rate or extent of hypoxia-inducible factor-1alpha signaling pathway. Sources: GOC:TermGenie, GOC:bf Also known as: regulation of HIF1alpha pathway, regulation of hypoxia-inducible factor-1alpha signalling pathway Relationships: is a type of regulation of intracellular signal transduction [GO:1902531]; regulates GO:0097411 Subtypes: negative regulation of hypoxia-inducible factor-1alpha signaling pathway [GO:1902072], positive regulation of hypoxia-inducible factor-1alpha signaling pathway [GO:1902073]